{
  "gene_symbol": "TADA2A",
  "term_label": "chromatin remodeling",
  "gene": "UniProtKB:O75478",
  "term_id": "GO:0006338",
  "gene_name": "Transcriptional adapter 2-alpha"
}